{
  "gene_name": "Arf-GAP with SH3 domain, ANK repeat and PH domain-containing protein 3",
  "gene": "UniProtKB:Q8TDY4",
  "gene_symbol": "ASAP3",
  "term_label": "focal adhesion",
  "term_id": "GO:0005925"
}